{
  "gene_name": "Junctophilin-3",
  "gene_symbol": "JPH3",
  "gene": "UniProtKB:Q8WXH2",
  "term_id": "GO:0048167",
  "term_label": "regulation of synaptic plasticity"
}